histone H4 methyltransferase activity [GO:0140939] (molecular function) Also known as: histone H4 methylase activity, histone H4 methylation References: PMID:28450737 Definition: Catalysis of the reaction: Catalysis of the reaction: S-adenosyl-L-methionine + a histone H4 = S-adenosyl-L-homocysteine + a methylated histone H4. Histone methylation generally occurs on either an arginine or a lysine residue. Relationships: is a type of GO:0042054 Subtypes: GO:0042799, GO:0044020, GO:0140984